{
  "term_id": "GO:0030258",
  "gene": "UniProtKB:Q6P1A2",
  "term_label": "lipid modification",
  "gene_symbol": "LPCAT3",
  "gene_name": "Lysophospholipid acyltransferase 5"
}